regulation of ATP metabolic process [GO:1903578] (biological process) Relationships: is a type of regulation of purine nucleotide metabolic process [GO:1900542]; regulates ATP metabolic process [GO:0046034] Also known as: regulation of ATP metabolism Subtypes: regulation of glycolytic process [GO:0006110], negative regulation of ATP metabolic process [GO:1903579], positive regulation of ATP metabolic process [GO:1903580], regulation of ATP biosynthetic process [GO:2001169] References: PMID:20695849 Sources: GOC:TermGenie, GO_REF:0000058 Definition: Any process that modulates the frequency, rate or extent of ATP metabolic process.